bone sialoprotein binding [GO:0044730] (molecular function) Also known as: bone sialoprotein II binding References: PMID:10642520 Definition: Binding to a bone sialoprotein, an extracellular matrix glycoprotein found on the surface of bones and dentin. Relationships: is a type of protein binding [GO:0005515]; is a type of extracellular matrix binding [GO:0050840]